toluene 4-monooxygenase activity [GO:0018638] (molecular function) References: PMID:15240250, PMID:36593585 Sources: RHEA:41380 Relationships: is_a oxidoreductase activity, acting on paired donors, with incorporation or reduction of molecular oxygen, NAD(P)H as one donor, and incorporation of one atom of oxygen [GO:0016709] Definition: Catalysis of the reaction: toluene + H+ + NADH + O2 = 4-methylphenol + H2O + NAD+.